determination of intestine left/right asymmetry [GO:0071908] (biological process) Sources: GOC:cvs Relationships: is a type of GO:0071907 Definition: Determination of the asymmetric location of the intestine loops with respect to the left and right halves of the organism.